{
  "gene_symbol": "RBCK1",
  "gene": "UniProtKB:Q9BYM8",
  "term_label": "proteasome-mediated ubiquitin-dependent protein catabolic process",
  "gene_name": "RanBP-type and C3HC4-type zinc finger-containing protein 1",
  "term_id": "GO:0043161"
}